glycolytic process from sucrose [GO:0061704] (biological process) Relationships: is a type of GO:0005987; is a type of glycolytic process [GO:0006096] References: PMID:15012287 Sources: GOC:dph, GOC:glycolysis Subtypes: GO:0061706 Definition: The chemical reactions and pathways resulting in the breakdown of a sucrose into pyruvate, with the concomitant production of a small amount of ATP and the reduction of NAD(P) to NAD(P)H. Glycolysis begins with the metabolism of a carbohydrate to generate products that can enter the pathway and ends with the production of pyruvate. Pyruvate may be converted to acetyl-coenzyme A, ethanol, lactate, or other small molecules.